{
  "gene": "UniProtKB:A0PJX2",
  "term_id": "GO:0005634",
  "gene_symbol": "TLDC2",
  "term_label": "nucleus",
  "gene_name": "TLD domain-containing protein 2"
}